{
  "term_label": "Unknown biological process",
  "term_id": "UNKNOWN:0002",
  "gene": "UniProtKB:O43909",
  "gene_name": "Exostosin-like 3",
  "gene_symbol": "EXTL3"
}